{
  "gene": "UniProtKB:Q12769",
  "term_label": "structural constituent of nuclear pore",
  "term_id": "GO:0017056",
  "gene_symbol": "NUP160",
  "gene_name": "Nuclear pore complex protein Nup160"
}